{
  "gene_name": "Arf-GAP with Rho-GAP domain, ANK repeat and PH domain-containing protein 1",
  "term_id": "GO:0005737",
  "gene": "UniProtKB:Q96P48",
  "term_label": "cytoplasm",
  "gene_symbol": "ARAP1"
}